{
  "gene_name": "Variable charge X-linked protein 3",
  "gene_symbol": "VCX3A",
  "term_id": "UNKNOWN:0003",
  "gene": "UniProtKB:Q9NNX9",
  "term_label": "Unknown cellular component"
}